{
  "gene_name": "Peroxisomal multifunctional enzyme type 2",
  "term_id": "GO:0005777",
  "gene_symbol": "HSD17B4",
  "term_label": "peroxisome",
  "gene": "UniProtKB:P51659"
}